{
  "term_id": "GO:0030154",
  "term_label": "cell differentiation",
  "gene_name": "Forkhead box protein D4-like 4",
  "gene_symbol": "FOXD4L4",
  "gene": "UniProtKB:Q8WXT5"
}